UDP-galactose-UDP-N-acetylglucosamine galactose phosphotransferase activity [GO:0047357] (molecular function) Definition: Catalysis of the reaction: UDP-N-acetyl-alpha-D-glucosamine + UDP-D-galactose = H+ + UDP-N-acetyl-6-(D-galactose-1-phospho)-D-glucosamine + UMP. Sources: EC:2.7.8.18, RHEA:22440 Also known as: UDP-galactose:UDP-N-acetyl-D-glucosamine galactose phosphotransferase activity, UDPgalactose-UDP-N-acetylglucosamine galactose phosphotransferase activity, UDPgalactose:UDP-N-acetyl-D-glucosamine galactose phosphotransferase activity, galactose-1-phosphotransferase activity, galactosyl phosphotransferase activity, uridine diphosphogalactose-uridine diphosphoacetylglucosamine galactose-1-phosphotransferase activity Relationships: is a type of GO:0016780